{
  "gene": "UniProtKB:Q8IUE0",
  "term_id": "GO:0000978",
  "term_label": "RNA polymerase II cis-regulatory region sequence-specific DNA binding",
  "gene_symbol": "TGIF2LY",
  "gene_name": "Homeobox protein TGIF2LY"
}